{
  "term_id": "GO:0004222",
  "gene_symbol": "MMP9",
  "gene": "UniProtKB:P14780",
  "gene_name": "Matrix metalloproteinase-9",
  "term_label": "metalloendopeptidase activity"
}